{
  "gene": "UniProtKB:Q9BY50",
  "gene_name": "Signal peptidase complex catalytic subunit SEC11C",
  "gene_symbol": "SEC11C",
  "term_id": "GO:0008233",
  "term_label": "peptidase activity"
}